{
  "gene_name": "Di-N-acetylchitobiase",
  "term_id": "GO:0009313",
  "term_label": "oligosaccharide catabolic process",
  "gene_symbol": "CTBS",
  "gene": "UniProtKB:Q01459"
}